{
  "gene_symbol": "EPX",
  "gene": "UniProtKB:P11678",
  "term_id": "GO:0042742",
  "gene_name": "Eosinophil peroxidase",
  "term_label": "defense response to bacterium"
}